pyruvate dehydrogenase (acetyl-transferring) kinase activity [GO:0004740] (molecular function) Definition: Catalysis of the reaction: ATP + L-seryl-[pyruvate dehydrogenase E1 alpha subunit] = ADP + H+ + O-phospho-L-seryl-[pyruvate dehydrogenase E1 alpha subunit]. Sources: RHEA:23052 Also known as: PDH kinase activity, PDHK, PDK, pyruvate dehydrogenase kinase (phosphorylating) activity, pyruvate dehydrogenase kinase activity Relationships: is a type of protein serine/threonine kinase activity [GO:0004674]